cyanelle ribonuclease P complex [GO:0030679] (cellular component) References: PMID:12045094 Sources: GOC:mah Also known as: cyanelle RNase P complex Definition: A ribonuclease P complex located in the cyanelle, where it catalyzes the 5' endonucleolytic cleavage of precursor tRNAs to yield mature tRNAs. The best characterized cyanelle ribonuclease P complex, from the alga Cyanophora paradoxa, contains a single RNA molecule that is necessary but not sufficient for catalysis, and several protein molecules. Relationships: is a type of multimeric ribonuclease P complex [GO:0030681]; is part of cyanelle [GO:0009842]